negative regulation of mast cell activation [GO:0033004] (biological process) Definition: Any process that stops, prevents, or reduces the frequency, rate, or extent of mast cell activation. Sources: GOC:mah Relationships: is_a negative regulation of leukocyte activation [GO:0002695]; is a type of regulation of mast cell activation [GO:0033003]; negatively regulates mast cell activation [GO:0045576] Subtypes: negative regulation of mast cell activation involved in immune response [GO:0033007]